{
  "gene_name": "Fragile X messenger ribonucleoprotein 1",
  "term_label": "regulation of mRNA stability",
  "gene": "UniProtKB:Q06787",
  "gene_symbol": "FMR1",
  "term_id": "GO:0043488"
}